tricetin O-methytransferase activity [GO:0102146] (molecular function) Sources: GOC:pz, RHEA:27493 Definition: Catalysis of the reaction: tricetin + S-adenosyl-L-methionine = H+ + 3'-O-methyltricetin + S-adenosyl-L-homocysteine. Relationships: is a type of GO:0008168